beta-D-galactofuranose catabolic process [GO:1901357] (biological process) Definition: The chemical reactions and pathways resulting in the breakdown of beta-D-galactofuranose. Also known as: beta-D-galactofuranose breakdown, beta-D-galactofuranose catabolism, beta-D-galactofuranose degradation Sources: GOC:TermGenie, GOC:di Relationships: is a type of galactose catabolic process [GO:0019388]